{
  "gene_name": "C-C motif chemokine 2",
  "gene_symbol": "CCL2",
  "term_label": "extracellular space",
  "gene": "UniProtKB:P13500",
  "term_id": "GO:0005615"
}